{
  "term_id": "GO:0042056",
  "gene_symbol": "VEGFB",
  "gene": "UniProtKB:P49765",
  "gene_name": "Vascular endothelial growth factor B",
  "term_label": "chemoattractant activity"
}